{
  "gene_symbol": "CDCA2",
  "gene_name": "Cell division cycle-associated protein 2",
  "gene": "UniProtKB:Q69YH5",
  "term_id": "GO:0005634",
  "term_label": "nucleus"
}